{
  "gene_symbol": "CILP2",
  "term_id": "UNKNOWN:0001",
  "gene_name": "Cartilage intermediate layer protein 2",
  "gene": "UniProtKB:Q8IUL8",
  "term_label": "Unknown molecular function"
}